axonemal outer doublet assembly [GO:0120308] (BP) Relationships: is a type of cellular component assembly [GO:0022607]; is part of axoneme assembly [GO:0035082] Definition: The aggregation, arrangement and bonding together of a set of components to form an axonemal outer doublet, a part of an axoneme consisting of a doublet microtubule. References: PMID:16278296 Sources: GOC:ach, GOC:krc Also known as: outer doublet assembly, outer-doublet microtubule assembly, axonemal outer doublet biogenesis, axonemal outer doublet formation, axonemal outer doublet morphogenesis, axoneme outer doublet assembly